mitotic spindle elongation (spindle phase three) [GO:0061805] (biological process) Also known as: mitotic anaphase spindle elongation, mitotic spindle elongation during anaphase, mitotic spindle elongation during mitotic anaphase Regulation: regulated by regulation of mitotic spindle elongation (spindle phase three) [GO:0110162]; negatively regulated by negative regulation of mitotic spindle elongation (spindle phase three) [GO:0110163]; positively regulated by positive regulation of mitotic spindle elongation (spindle phase three) [GO:0110164] Relationships: is a type of mitotic spindle organization [GO:0007052]; is part of mitotic spindle elongation [GO:0000022]; happens during mitotic anaphase B [GO:0000092] References: PMID:21920317 Sources: GOC:dph, GOC:vw Definition: The cell cycle process in which the distance is lengthened between poles of the mitotic spindle during mitotic anaphase B.